{
  "gene_name": "Dedicator of cytokinesis protein 10",
  "gene_symbol": "DOCK10",
  "term_id": "UNKNOWN:0003",
  "term_label": "Unknown cellular component",
  "gene": "UniProtKB:Q96BY6"
}